{
  "gene_name": "DNA topoisomerase 2-beta",
  "term_label": "resolution of meiotic recombination intermediates",
  "term_id": "GO:0000712",
  "gene_symbol": "TOP2B",
  "gene": "UniProtKB:Q02880"
}